{
  "term_id": "GO:0005771",
  "gene_symbol": "CHMP1B",
  "gene": "UniProtKB:Q7LBR1",
  "term_label": "multivesicular body",
  "gene_name": "Charged multivesicular body protein 1b"
}